regulation of epidermis development [GO:0045682] (biological process) Also known as: regulation of epidermal development, regulation of hypodermis development Definition: Any process that modulates the frequency, rate or extent of epidermis development. Relationships: is a type of regulation of developmental process [GO:0050793]; regulates epidermis development [GO:0008544] Subtypes: regulation of epidermal cell differentiation [GO:0045604], negative regulation of epidermis development [GO:0045683], positive regulation of epidermis development [GO:0045684] Sources: GOC:go_curators